old growing cell tip [GO:0035840] (cellular component) Definition: A cell tip which has existed for at least one complete cell cycle, and at which polarized growth occurs. For example, in fission yeast the cell end that existed prior to cell division grows immediately after division, and contains a distinctive complement of proteins including actin cytoskeletal structures. Sources: GOC:expert_jd, GOC:mah Also known as: old growing cell end Relationships: is a type of growing cell tip [GO:0035838] Subtypes: old cell tip after activation of bipolar cell growth [GO:0035842]